{
  "gene_symbol": "INPP5K",
  "term_id": "GO:0043005",
  "term_label": "neuron projection",
  "gene_name": "Inositol polyphosphate 5-phosphatase K",
  "gene": "UniProtKB:Q9BT40"
}